{
  "term_id": "GO:0005737",
  "gene_symbol": "GAK",
  "term_label": "cytoplasm",
  "gene_name": "Cyclin-G-associated kinase",
  "gene": "UniProtKB:O14976"
}